G protein-coupled receptor internalization [GO:0002031] (biological process) References: PMID:8396717 Also known as: G-protein coupled receptor internalization Subtypes: prostaglandin receptor internalization [GO:1990767] Definition: The process that results in the uptake of a G protein-coupled receptor into an endocytic vesicle. Relationships: is a type of receptor internalization [GO:0031623]; is part of desensitization of G protein-coupled receptor signaling pathway [GO:0002029] Regulation: regulated by regulation of G protein-coupled receptor internalization [GO:1904020]; negatively regulated by negative regulation of G protein-coupled receptor internalization [GO:1904021]; positively regulated by positive regulation of G protein-coupled receptor internalization [GO:1904022]